{
  "gene_name": "Complexin-1",
  "gene": "UniProtKB:O14810",
  "gene_symbol": "CPLX1",
  "term_id": "GO:0000149",
  "term_label": "SNARE binding"
}